multivesicular body assembly [GO:0036258] (biological process) Definition: The aggregation, arrangement and bonding together of a set of components to form a multivesicular body, a type of late endosome in which regions of the limiting endosomal membrane invaginate to form internal vesicles; membrane proteins that enter the internal vesicles are sequestered from the cytoplasm. References: PMID:11566881, PMID:19571114 Sources: GOC:sart Also known as: MVB biogenesis, MVB formation, multivesicular body biogenesis Relationships: is a type of multivesicular body organization [GO:0036257]; is a type of organelle assembly [GO:0070925]